{
  "gene_name": "Serine_arginine repetitive matrix protein 2",
  "term_id": "UNKNOWN:0003",
  "gene_symbol": "SRRM2",
  "gene": "UniProtKB:Q9UQ35",
  "term_label": "Unknown cellular component"
}